{
  "term_id": "UNKNOWN:0002",
  "term_label": "Unknown biological process",
  "gene": "UniProtKB:Q9NV79",
  "gene_symbol": "PCMTD2",
  "gene_name": "Protein-L-isoaspartate O-methyltransferase domain-containing protein 2"
}